{
  "gene_name": "Cation channel sperm-associated auxiliary subunit beta",
  "gene": "UniProtKB:Q9H7T0",
  "gene_symbol": "CATSPERB",
  "term_id": "GO:0036128",
  "term_label": "CatSper complex"
}